{
  "gene_symbol": "P2RX1",
  "gene": "UniProtKB:P51575",
  "term_id": "GO:0070588",
  "term_label": "calcium ion transmembrane transport",
  "gene_name": "P2X purinoceptor 1"
}